male pronucleus assembly [GO:0035039] (biological process) References: PMID:11735001 Sources: GOC:bf Definition: The conversion at fertilization of the inactive sperm nucleus into a male pronucleus with its chromosomes processed for the first zygotic division. Also known as: male pronucleus formation Relationships: is a type of nucleus organization [GO:0006997]; is a type of GO:0070925; is part of single fertilization [GO:0007338]